{
  "gene_name": "AFG3-like protein 2",
  "gene_symbol": "AFG3L2",
  "term_label": "metalloendopeptidase activity",
  "term_id": "GO:0004222",
  "gene": "UniProtKB:Q9Y4W6"
}